{
  "gene": "UniProtKB:Q9HA65",
  "gene_symbol": "TBC1D17",
  "term_label": "cytosol",
  "gene_name": "TBC1 domain family member 17",
  "term_id": "GO:0005829"
}